{
  "gene_symbol": "LIM2",
  "gene_name": "Lens fiber membrane intrinsic protein",
  "term_label": "plasma membrane",
  "gene": "UniProtKB:P55344",
  "term_id": "GO:0005886"
}